{
  "gene": "UniProtKB:P00966",
  "term_label": "L-arginine biosynthetic process",
  "gene_symbol": "ASS1",
  "gene_name": "Argininosuccinate synthase",
  "term_id": "GO:0006526"
}